{
  "term_label": "T cell receptor signaling pathway",
  "term_id": "GO:0050852",
  "gene": "UniProtKB:Q5ZPR3",
  "gene_name": "CD276 antigen",
  "gene_symbol": "CD276"
}